{
  "term_label": "chromatin binding",
  "gene_symbol": "SMC2",
  "gene": "UniProtKB:O95347",
  "gene_name": "Structural maintenance of chromosomes protein 2",
  "term_id": "GO:0003682"
}